{
  "term_id": "UNKNOWN:0002",
  "gene": "UniProtKB:Q11128",
  "term_label": "Unknown biological process",
  "gene_symbol": "FUT5",
  "gene_name": "4-galactosyl-N-acetylglucosaminide 3-alpha-L-fucosyltransferase FUT5"
}